{
  "gene_name": "NADH dehydrogenase [ubiquinone] 1 alpha subcomplex subunit 2",
  "gene": "UniProtKB:O43678",
  "term_label": "Unknown biological process",
  "gene_symbol": "NDUFA2",
  "term_id": "UNKNOWN:0002"
}